{
  "gene": "UniProtKB:P60369",
  "gene_name": "Keratin-associated protein 10-3",
  "term_id": "UNKNOWN:0001",
  "term_label": "Unknown molecular function",
  "gene_symbol": "KRTAP10-3"
}